{
  "gene_name": "Bone morphogenetic protein 4",
  "term_id": "GO:0005615",
  "term_label": "extracellular space",
  "gene": "UniProtKB:P12644",
  "gene_symbol": "BMP4"
}